{
  "gene_symbol": "LBX1",
  "term_id": "GO:1990837",
  "gene": "UniProtKB:P52954",
  "term_label": "sequence-specific double-stranded DNA binding",
  "gene_name": "Transcription factor LBX1"
}